{
  "term_label": "UDP phosphatase activity",
  "gene_symbol": "ENTPD3",
  "gene": "UniProtKB:O75355",
  "gene_name": "Ectonucleoside triphosphate diphosphohydrolase 3",
  "term_id": "GO:0045134"
}